{
  "term_label": "G protein-coupled receptor signaling pathway",
  "gene_name": "P2Y purinoceptor 12",
  "gene_symbol": "P2RY12",
  "term_id": "GO:0007186",
  "gene": "UniProtKB:Q9H244"
}